{
  "gene_name": "Hippocampus abundant transcript-like protein 1",
  "gene_symbol": "MFSD14B",
  "gene": "UniProtKB:Q5SR56",
  "term_id": "UNKNOWN:0001",
  "term_label": "Unknown molecular function"
}